killing by host of symbiont cells [GO:0051873] (biological process) Sources: GOC:add Definition: Any process mediated by an organism that results in the death of cells in the symbiont organism. The symbiont is defined as the smaller of the organisms involved in a symbiotic interaction. Relationships: is_a GO:0031640; is a type of biological process involved in interaction with symbiont [GO:0051702]; is a type of defense response to symbiont [GO:0140546] Also known as: disruption by host of symbiont cells Subtypes: GO:0051838, neutrophil-mediated killing of symbiont cell [GO:0070943]